{
  "term_id": "UNKNOWN:0003",
  "gene_symbol": "CCDC117",
  "gene": "UniProtKB:Q8IWD4",
  "gene_name": "Coiled-coil domain-containing protein 117",
  "term_label": "Unknown cellular component"
}